CBM complex [GO:0032449] (cellular component) Relationships: is a type of intracellular protein-containing complex [GO:0140535] References: PMID:12909454, PMID:30467369 Also known as: CARMA1-BCL10-Malt1 complex Definition: A protein complex comprising Bcl10, MALT1 and a CARD domain-containing protein (CARD9, CARD10 or CARD11); plays a role in signal transduction during NF-kappaB activation.